methylglyoxal reductase (NADH) activity [GO:0019170] (MF) Also known as: D-lactaldehyde dehydrogenase activity, methylglyoxal reductase (NADH-dependent) activity, methylglyoxal reductase activity, (R)-lactaldehyde:NAD+ oxidoreductase activity Definition: Catalysis of the reaction: (R)-lactaldehyde + NAD+ = methylglyoxal + NADH + H+. Relationships: is a type of oxidoreductase activity, acting on the CH-OH group of donors, NAD or NADP as acceptor [GO:0016616] Sources: EC:1.1.1.78